negative regulation of telomeric loop formation [GO:1904419] (biological process) Definition: Any process that stops, prevents or reduces the frequency, rate or extent of telomeric loop formation. References: PMID:22579284 Sources: GOC:BHF, GOC:BHF_telomere, GOC:TermGenie, GOC:nc, GO_REF:0000058 Also known as: down regulation of t-loop biosynthesis, down regulation of t-loop formation, down regulation of telomeric loop formation, down-regulation of t-loop biosynthesis, down-regulation of t-loop formation, down-regulation of telomeric loop formation, downregulation of t-loop biosynthesis, downregulation of t-loop formation, downregulation of telomeric loop formation, negative regulation of t-loop biosynthesis, negative regulation of t-loop formation, inhibition of t-loop biosynthesis, inhibition of t-loop formation, inhibition of telomeric loop formation Relationships: is a type of negative regulation of telomere maintenance [GO:0032205]; is a type of regulation of telomeric loop formation [GO:1904418]; negatively regulates telomeric loop formation [GO:0031627]